{
  "gene_symbol": "CPNE1",
  "gene": "UniProtKB:Q99829",
  "gene_name": "Copine-1",
  "term_id": "GO:1903265",
  "term_label": "positive regulation of tumor necrosis factor-mediated signaling pathway"
}